{
  "gene_symbol": "NWD2",
  "gene_name": "NACHT and WD repeat domain-containing protein 2",
  "term_id": "UNKNOWN:0001",
  "term_label": "Unknown molecular function",
  "gene": "UniProtKB:Q9ULI1"
}